{
  "term_label": "Unknown molecular function",
  "gene_symbol": "TDH",
  "gene": "UniProtKB:Q8IZJ6",
  "gene_name": "Inactive L-threonine 3-dehydrogenase, mitochondrial",
  "term_id": "UNKNOWN:0001"
}